{
  "term_id": "GO:0005634",
  "gene_symbol": "BHLHE22",
  "term_label": "nucleus",
  "gene_name": "Class E basic helix-loop-helix protein 22",
  "gene": "UniProtKB:Q8NFJ8"
}